{
  "term_id": "UNKNOWN:0003",
  "gene_name": "Alpha-aminoadipic semialdehyde dehydrogenase",
  "gene": "UniProtKB:P49419",
  "gene_symbol": "ALDH7A1",
  "term_label": "Unknown cellular component"
}